{
  "gene_name": "Protein Wnt-9b",
  "gene": "UniProtKB:O14905",
  "term_id": "GO:0030182",
  "term_label": "neuron differentiation",
  "gene_symbol": "WNT9B"
}